{
  "gene_symbol": "TLX3",
  "term_label": "regulation of transcription by RNA polymerase II",
  "gene": "UniProtKB:O43711",
  "term_id": "GO:0006357",
  "gene_name": "T-cell leukemia homeobox protein 3"
}